{
  "gene": "UniProtKB:Q9UJU6",
  "gene_name": "Drebrin-like protein",
  "term_id": "GO:0030674",
  "gene_symbol": "DBNL",
  "term_label": "protein-macromolecule adaptor activity"
}